{
  "gene_symbol": "SETSIP",
  "term_label": "chromatin binding",
  "gene_name": "Protein SETSIP",
  "term_id": "GO:0003682",
  "gene": "UniProtKB:P0DME0"
}